neoxanthin synthase activity [GO:0034020] (molecular function) Sources: EC:5.3.99.9, RHEA:10128 Relationships: is a type of intramolecular oxidoreductase activity [GO:0016860] Also known as: NSY, violaxanthin-neoxanthin isomerase (epoxide-opening) activity Definition: Catalysis of the reaction: all-trans-violaxanthin = all-trans-neoxanthin.